{
  "gene_name": "Protein Aster-C",
  "term_id": "GO:0140268",
  "gene": "UniProtKB:Q8IYS0",
  "term_label": "endoplasmic reticulum-plasma membrane contact site",
  "gene_symbol": "GRAMD1C"
}